{
  "term_id": "GO:0004060",
  "gene_symbol": "NAT1",
  "gene": "UniProtKB:P18440",
  "gene_name": "Arylamine N-acetyltransferase 1",
  "term_label": "arylamine N-acetyltransferase activity"
}